{
  "gene": "UniProtKB:P22033",
  "term_label": "cytoplasm",
  "gene_name": "Methylmalonyl-CoA mutase, mitochondrial",
  "gene_symbol": "MMUT",
  "term_id": "GO:0005737"
}